{
  "gene": "UniProtKB:Q9UL59",
  "gene_symbol": "ZNF214",
  "term_label": "Unknown biological process",
  "term_id": "UNKNOWN:0002",
  "gene_name": "Zinc finger protein 214"
}